{
  "term_label": "Unknown cellular component",
  "gene_symbol": "OR5A2",
  "gene_name": "Olfactory receptor 5A2",
  "gene": "UniProtKB:Q8NGI9",
  "term_id": "UNKNOWN:0003"
}